{
  "term_label": "Unknown cellular component",
  "term_id": "UNKNOWN:0003",
  "gene": "UniProtKB:Q8NAC3",
  "gene_name": "Interleukin-17 receptor C",
  "gene_symbol": "IL17RC"
}